{
  "gene_symbol": "ENSA",
  "term_id": "UNKNOWN:0002",
  "gene_name": "Alpha-endosulfine",
  "term_label": "Unknown biological process",
  "gene": "UniProtKB:O43768"
}